{
  "term_id": "UNKNOWN:0003",
  "gene_symbol": "KRTCAP3",
  "gene_name": "Keratinocyte-associated protein 3",
  "term_label": "Unknown cellular component",
  "gene": "UniProtKB:Q53RY4"
}